{
  "term_label": "DNA-binding transcription factor activity, RNA polymerase II-specific",
  "gene": "UniProtKB:Q99801",
  "term_id": "GO:0000981",
  "gene_name": "Homeobox protein Nkx-3.1",
  "gene_symbol": "NKX3-1"
}